{
  "term_label": "alcohol-forming very long-chain fatty acyl-CoA reductase activity",
  "gene_symbol": "FAR1",
  "gene_name": "Fatty acyl-CoA reductase 1",
  "gene": "UniProtKB:Q8WVX9",
  "term_id": "GO:0080019"
}